{
  "term_id": "GO:0050821",
  "term_label": "protein stabilization",
  "gene": "UniProtKB:Q99933",
  "gene_name": "BAG family molecular chaperone regulator 1",
  "gene_symbol": "BAG1"
}